Gemin6-Gemin7-unrip complex [GO:0034717] (CC) Relationships: is a type of intracellular protein-containing complex [GO:0140535] Definition: A protein complex that contains Gemin6, Gemin7, and unrip (STRAP), and can bind to snRNAs; may play a role in snRNP assembly. References: PMID:17640873 Sources: GOC:mah